{
  "gene_symbol": "FARSB",
  "gene_name": "Phenylalanine--tRNA ligase beta subunit",
  "term_label": "phenylalanine-tRNA ligase complex",
  "term_id": "GO:0009328",
  "gene": "UniProtKB:Q9NSD9"
}